{
  "gene_name": "Actin-like protein 6A",
  "gene_symbol": "ACTL6A",
  "term_label": "NuA4 histone acetyltransferase complex",
  "gene": "UniProtKB:O96019",
  "term_id": "GO:0035267"
}